phenylserine aldolase activity [GO:0050179] (MF) Sources: EC:4.1.2.26, RHEA:21712 Also known as: L-threo-3-phenylserine benzaldehyde-lyase (glycine-forming), L-threo-3-phenylserine benzaldehyde-lyase activity Definition: Catalysis of the reaction: L-threo-3-phenylserine = benzaldehyde + glycine. Relationships: is_a aldehyde-lyase activity [GO:0016832]